multivesicular body [GO:0005771] (CC) Relationships: is a type of GO:0005770 References: PMID:11566881, PMID:16533950 Also known as: MVB, MVE, multivesicular endosome Definition: A type of endosome in which regions of the limiting endosomal membrane invaginate to form internal vesicles; membrane proteins that enter the internal vesicles are sequestered from the cytoplasm.